{
  "gene_symbol": "ATG7",
  "gene": "UniProtKB:O95352",
  "gene_name": "Ubiquitin-like modifier-activating enzyme ATG7",
  "term_label": "Atg8 activating enzyme activity",
  "term_id": "GO:0019779"
}